{
  "gene_name": "Autophagy protein 5",
  "gene": "UniProtKB:Q9H1Y0",
  "gene_symbol": "ATG5",
  "term_label": "cellular response to nitrogen starvation",
  "term_id": "GO:0006995"
}